{
  "term_label": "Unknown biological process",
  "gene_name": "Leucine-rich repeat and transmembrane domain-containing protein 1",
  "term_id": "UNKNOWN:0002",
  "gene": "UniProtKB:Q9HBL6",
  "gene_symbol": "LRTM1"
}